operant conditioning [GO:0035106] (biological process) Definition: Learning to anticipate future events on the basis of past experience with the consequences of one's own behavior. References: PMID:14662373 Also known as: instrumental conditioning Relationships: is a type of GO:0007612